{
  "term_id": "GO:0000398",
  "gene_symbol": "SART3",
  "gene_name": "Squamous cell carcinoma antigen recognized by T-cells 3",
  "term_label": "mRNA splicing, via spliceosome",
  "gene": "UniProtKB:Q15020"
}